protease localization to mast cell secretory granule [GO:0033368] (biological process) Also known as: protease localisation in mast cell secretory granule, protease localization in mast cell secretory granule Definition: Any process in which a protease is transported to, or maintained in, a location within a secretory granule in a mast cell. Sources: GOC:mah Relationships: is a type of protein localization to mast cell secretory granule [GO:0033367]